cyclin-dependent protein serine/threonine kinase regulator activity [GO:0016538] (molecular function) Also known as: cyclin, cyclin-dependent protein kinase regulator activity, G1/S-specific cyclin, G2/M-specific cyclin, cyclin-dependent protein kinase, intrinsic regulator activity References: PMID:7877684, PMID:9442875 Sources: GOC:pr, GOC:rn Subtypes: cyclin-dependent protein serine/threonine kinase inhibitor activity [GO:0004861], cyclin-dependent protein serine/threonine kinase activator activity [GO:0061575] Definition: Modulates the activity of a cyclin-dependent protein serine/threonine kinase, enzymes of the protein kinase family that are regulated through association with cyclins and other proteins. Relationships: is a type of cyclin-dependent protein kinase regulator activity [GO:0019914]; regulates cyclin-dependent protein serine/threonine kinase activity [GO:0004693]